hyaluranon cable [GO:0036117] (cellular component) Definition: A cable structure, surrounding some cell types (e.g. proximal or bronchial tubular epithelial cells), and composed of hyaluranon (HA), a ubiquitous connective tissue glycosaminoglycan. References: PMID:16900089 Sources: GOC:yaf Also known as: HA cable Relationships: is a type of cellular anatomical structure [GO:0110165]; is part of extracellular region [GO:0005576]